{
  "gene_name": "Carabin",
  "term_label": "GTPase activator activity",
  "term_id": "GO:0005096",
  "gene": "UniProtKB:Q8IV04",
  "gene_symbol": "TBC1D10C"
}